{
  "term_id": "GO:0007507",
  "term_label": "heart development",
  "gene": "UniProtKB:Q9NPF8",
  "gene_name": "Arf-GAP with dual PH domain-containing protein 2",
  "gene_symbol": "ADAP2"
}